carnitine transport [GO:0015879] (biological process) Relationships: is a type of GO:0015695; is a type of amino-acid betaine transport [GO:0015838] Also known as: vitamin Bt transport Subtypes: (R)-carnitine transport [GO:1900749], carnitine transmembrane transport [GO:1902603] Sources: GOC:ai Definition: The directed movement of carnitine into, out of or within a cell, or between cells, by means of some agent such as a transporter or pore. Carnitine is a compound that participates in the transfer of acyl groups across the inner mitochondrial membrane.